alpha-1A adrenergic receptor binding [GO:0031691] (molecular function) Definition: Binding to an alpha-1A adrenergic receptor. Relationships: is a type of adrenergic receptor binding [GO:0031690] Also known as: alpha-1A adrenergic receptor ligand Sources: GOC:mah, GOC:nln